{
  "term_label": "semaphorin receptor activity",
  "gene_name": "Plexin-D1",
  "gene": "UniProtKB:Q9Y4D7",
  "term_id": "GO:0017154",
  "gene_symbol": "PLXND1"
}